manchette [GO:0002177] (cellular component) Definition: A tubular array of microtubules that extends from the perinuclear ring surrounding the spermatid nucleus to the flagellar axoneme. The manchette may also contain F-actin filaments. References: PMID:15018141, PMID:22319670, PMID:24440897, PMID:26792866 Sources: GOC:krc Relationships: is a type of cellular anatomical structure [GO:0110165]; is part of GO:0015630